{
  "gene": "UniProtKB:Q96M78",
  "gene_symbol": "FER1L6-AS2",
  "gene_name": "Putative uncharacterized protein encoded by FER1L6-AS2",
  "term_label": "Unknown cellular component",
  "term_id": "UNKNOWN:0003"
}